{
  "gene_name": "Neuralized-like protein 4",
  "term_label": "Unknown biological process",
  "gene": "UniProtKB:Q96JN8",
  "gene_symbol": "NEURL4",
  "term_id": "UNKNOWN:0002"
}